{
  "term_id": "GO:0005634",
  "gene_name": "Homeobox protein Hox-B2",
  "gene": "UniProtKB:P14652",
  "gene_symbol": "HOXB2",
  "term_label": "nucleus"
}